mating-type M-factor pheromone receptor activity [GO:0036319] (molecular function) References: PMID:7941744 Sources: GOC:al Also known as: M-factor mating pheromone receptor activity, M-factor receptor activity Relationships: is a type of mating-type factor pheromone receptor activity [GO:0004932]; is a type of GO:0036318 Definition: Combining with the mating-type peptide pheromone M-factor and transmitting the signal across the membrane to initiate a change in cell activity. M-factor is a nine-membered oligopeptide that consists of tyrosyl, threonyl, prolyl, lysyl, valyl, prolyl, tyrosyl, methionyl and methyl S-farnesylcysteinate residues joined in sequence, and is a peptide pheromone released by Schizosaccharomyces pombe cells of the cellular mating type Minus.